{
  "gene_symbol": "TRAJ52",
  "gene": "UniProtKB:A0A075B6W2",
  "gene_name": "T cell receptor alpha joining 52 (Fragment)",
  "term_id": "UNKNOWN:0003",
  "term_label": "Unknown cellular component"
}